motile cilium [GO:0031514] (cellular component) Definition: A cilium which may have a variable arrangement of axonemal microtubules and also contains molecular motors. It may beat with a whip-like pattern that promotes cell motility or transport of fluids and other cells across a cell surface, such as on epithelial cells that line the lumenal ducts of various tissues; or they may display a distinct twirling motion that directs fluid flow asymmetrically across the cellular surface to affect asymmetric body plan organization. Motile cilia can be found in single as well as multiple copies per cell. Also known as: motile cilia, microtubule-based flagellum, motile primary cilia, motile primary cilium, motile secondary cilium, nodal cilium Relationships: is_a cilium [GO:0005929] References: PMID:17009929, PMID:20144998, PMID:22118931 Sources: GOC:cilia, GOC:dgh, GOC:kmv Subtypes: 9+0 motile cilium [GO:0097728], GO:0097729